GBAF complex [GO:0140288] (cellular component) References: PMID:29374058 Relationships: is a type of GO:0070603 Definition: A SWI/SNF subcomplex that incorporates two mutually exclusive paralogs, GLTSCR1 (glioma tumor suppressor candidate region gene 1) or GLTSCR1L (GLTSCR1-like), BRD9 (bromodomain-containing 9) and the BAF subunits BAF155, BAF60, SS18, BAF53a, and BRG1/BRM.